{
  "term_label": "regulation of membrane potential",
  "gene": "UniProtKB:Q8NCM2",
  "gene_symbol": "KCNH5",
  "term_id": "GO:0042391",
  "gene_name": "Potassium voltage-gated channel subfamily H member 5"
}